midbrain-hindbrain boundary maturation during brain development [GO:0022004] (biological process) References: PMID:15541513 Sources: GOC:cls, GOC:dgh, GOC:dph, GOC:jid, GO_REF:0000021 Definition: A developmental process occurring after the brain has been specified along the neural axis that is required for the midbrain-hindbrain boundary to attain its fully functional state. The midbrain-hindbrain domain of the embryonic brain is comprised of the mesencephalic vesicle and the first rhombencephalic vesicle at early somitogenesis stages. An organizing center at the boundary patterns the midbrain and hindbrain primordia of the neural plate. Relationships: is_a multicellular organismal process [GO:0032501]; is part of midbrain-hindbrain boundary maturation [GO:0021732]